{
  "gene_name": "Cadherin-13",
  "gene": "UniProtKB:P55290",
  "term_label": "adherens junction organization",
  "gene_symbol": "CDH13",
  "term_id": "GO:0034332"
}